{
  "gene_name": "Putative protein CDKN2A-DT",
  "gene": "UniProtKB:Q9UH64",
  "gene_symbol": "CDKN2A-DT",
  "term_label": "Unknown biological process",
  "term_id": "UNKNOWN:0002"
}